{
  "gene": "UniProtKB:Q13410",
  "gene_symbol": "BTN1A1",
  "term_label": "signaling receptor binding",
  "term_id": "GO:0005102",
  "gene_name": "Butyrophilin subfamily 1 member A1"
}